{
  "term_id": "GO:0005886",
  "gene": "UniProtKB:Q8NFF2",
  "term_label": "plasma membrane",
  "gene_name": "Sodium_potassium_calcium exchanger 4",
  "gene_symbol": "SLC24A4"
}